{
  "term_label": "sequence-specific DNA binding",
  "gene_name": "Myelin regulatory factor-like protein",
  "gene_symbol": "MYRFL",
  "gene": "UniProtKB:Q96LU7",
  "term_id": "GO:0043565"
}